{
  "gene_name": "Aryl-hydrocarbon-interacting protein-like 1",
  "gene": "UniProtKB:Q9NZN9",
  "gene_symbol": "AIPL1",
  "term_label": "Unknown biological process",
  "term_id": "UNKNOWN:0002"
}